{
  "term_label": "Unknown biological process",
  "gene_symbol": "SLC16A13",
  "gene_name": "Monocarboxylate transporter 13",
  "term_id": "UNKNOWN:0002",
  "gene": "UniProtKB:Q7RTY0"
}